{
  "term_label": "canonical NF-kappaB signal transduction",
  "gene": "UniProtKB:Q01201",
  "gene_name": "Transcription factor RelB",
  "gene_symbol": "RELB",
  "term_id": "GO:0007249"
}